{
  "gene": "UniProtKB:P09417",
  "term_label": "cytoplasm",
  "gene_symbol": "QDPR",
  "term_id": "GO:0005737",
  "gene_name": "Dihydropteridine reductase"
}